{
  "term_id": "UNKNOWN:0003",
  "gene_symbol": "TNFRSF9",
  "gene_name": "Tumor necrosis factor receptor superfamily member 9",
  "term_label": "Unknown cellular component",
  "gene": "UniProtKB:Q07011"
}